stromal-epithelial cell signaling involved in prostate gland development [GO:0044345] (BP) Also known as: stromal-epithelial cell signalling involved in prostate gland development Definition: The process of transferring information from a stromal cell to an epithelial cell where it is received and interpreted, as part of prostate gland development. Sources: GOC:jl, GOC:yaf Relationships: is a type of cell-cell signaling [GO:0007267]; is a type of cellular process involved in reproduction in multicellular organism [GO:0022412]; is part of prostate gland development [GO:0030850]